{
  "gene_name": "Acetyl-coenzyme A thioesterase",
  "term_id": "GO:0006084",
  "gene_symbol": "ACOT12",
  "gene": "UniProtKB:Q8WYK0",
  "term_label": "acetyl-CoA metabolic process"
}